{
  "term_id": "GO:0005886",
  "gene_symbol": "LRRTM4",
  "gene_name": "Leucine-rich repeat transmembrane neuronal protein 4",
  "term_label": "plasma membrane",
  "gene": "UniProtKB:Q86VH4"
}